{
  "gene_symbol": "USP17L19",
  "gene_name": "Ubiquitin carboxyl-terminal hydrolase 17-like protein 19",
  "term_label": "cysteine-type deubiquitinase activity",
  "gene": "UniProtKB:D6RCP7",
  "term_id": "GO:0004843"
}